{
  "gene_name": "Transmembrane protein 269",
  "gene": "UniProtKB:A0A1B0GVZ9",
  "term_id": "UNKNOWN:0002",
  "term_label": "Unknown biological process",
  "gene_symbol": "TMEM269"
}